siderophore transport [GO:0015891] (biological process) Definition: The directed movement of siderophores, low molecular weight Fe(III)-chelating substances, into, out of or within a cell, or between cells, by means of some agent such as a transporter or pore. Relationships: is a type of GO:1901678 Also known as: iron-siderophore transport, siderophore-iron transport, iron-siderochrome transport, siderochrome transport Sources: GOC:ai Subtypes: enterobactin transport [GO:0042930], chrysobactin transport [GO:0042932], achromobactin transport [GO:0042935], GO:0044718